{
  "gene_name": "Poly(rC)-binding protein 2",
  "term_label": "nucleus",
  "gene": "UniProtKB:Q15366",
  "gene_symbol": "PCBP2",
  "term_id": "GO:0005634"
}